{
  "term_id": "GO:0044331",
  "gene_name": "Cadherin-24",
  "term_label": "cell-cell adhesion mediated by cadherin",
  "gene_symbol": "CDH24",
  "gene": "UniProtKB:Q86UP0"
}